{
  "gene": "UniProtKB:Q8N9V6",
  "gene_name": "Ankyrin repeat domain-containing protein 53",
  "gene_symbol": "ANKRD53",
  "term_id": "GO:0000922",
  "term_label": "spindle pole"
}